{
  "gene": "UniProtKB:Q9Y5J3",
  "term_id": "GO:0000122",
  "gene_name": "Hairy_enhancer-of-split related with YRPW motif protein 1",
  "term_label": "negative regulation of transcription by RNA polymerase II",
  "gene_symbol": "HEY1"
}